{
  "gene_symbol": "EHMT2",
  "gene_name": "Histone-lysine N-methyltransferase EHMT2",
  "term_id": "GO:0000122",
  "gene": "UniProtKB:Q96KQ7",
  "term_label": "negative regulation of transcription by RNA polymerase II"
}